{
  "term_id": "GO:0032502",
  "gene": "UniProtKB:Q7RTU0",
  "gene_name": "Transcription factor 24",
  "term_label": "developmental process",
  "gene_symbol": "TCF24"
}